{
  "gene": "UniProtKB:Q8NCW6",
  "gene_symbol": "GALNT11",
  "term_label": "regulation of Notch signaling pathway",
  "term_id": "GO:0008593",
  "gene_name": "Polypeptide N-acetylgalactosaminyltransferase 11"
}